{
  "gene_symbol": "TRBV5-3",
  "gene": "UniProtKB:A0A0A0MS03",
  "term_id": "UNKNOWN:0001",
  "gene_name": "Probable non-functional T cell receptor beta variable 5-3",
  "term_label": "Unknown molecular function"
}